positive regulation of acetylcholine metabolic process [GO:0060409] (biological process) Definition: Any process that increases the rate, frequency or extent of the chemical reactions and pathways involving acetylcholine, the acetic acid ester of the organic base choline. Acetylcholine is a major neurotransmitter and neuromodulator both in the central and peripheral nervous systems. It also acts as a paracrine signal in various non-neural tissues. Sources: GOC:dph, GOC:tb Relationships: is a type of positive regulation of amine metabolic process [GO:0033240]; is a type of regulation of acetylcholine metabolic process [GO:0060408]; positively regulates acetylcholine metabolic process [GO:0008291] Subtypes: positive regulation of acetylcholine biosynthetic process [GO:1905923]